{
  "gene_symbol": "LUC7L3",
  "gene": "UniProtKB:O95232",
  "term_id": "GO:0003729",
  "gene_name": "Luc7-like protein 3",
  "term_label": "mRNA binding"
}